(S)-2-hydroxy-acid oxidase activity [GO:0003973] (molecular function) Also known as: hydroxy-acid oxidase A activity, hydroxy-acid oxidase B activity, long-chain-(S)-2-hydroxy-long-chain-acid oxidase activity, medium-chain-(S)-2-hydroxy-acid oxidase activity, very-long-chain-(S)-2-hydroxy-acid oxidase activity, L-2-hydroxy acid oxidase, L-alpha-hydroxy acid oxidase, glycolate oxidase activity, hydroxyacid oxidase A Relationships: is a type of oxidoreductase activity, acting on the CH-OH group of donors, oxygen as acceptor [GO:0016899] Definition: Catalysis of the reaction: (S)-2-hydroxy-acid + O2 = 2-oxo acid + hydrogen peroxide. Sources: RHEA:16789